{
  "term_id": "GO:0005886",
  "gene_symbol": "ARC",
  "gene_name": "Activity-regulated cytoskeleton-associated protein",
  "gene": "UniProtKB:Q7LC44",
  "term_label": "plasma membrane"
}